{
  "term_label": "intracellular calcium ion homeostasis",
  "gene_name": "Endothelin-3",
  "gene": "UniProtKB:P14138",
  "term_id": "GO:0006874",
  "gene_symbol": "EDN3"
}